type 2 orexin receptor binding [GO:0031772] (molecular function) Definition: Binding to a type 2 orexin receptor. Sources: GOC:mah, GOC:nln Also known as: OX2 orexin receptor binding, type 2 hypocretin receptor binding, type 2 hypocretin receptor ligand Relationships: is a type of orexin receptor binding [GO:0042324]